{
  "term_label": "peptide binding",
  "gene_name": "NACHT, LRR and PYD domains-containing protein 6",
  "gene_symbol": "NLRP6",
  "gene": "UniProtKB:P59044",
  "term_id": "GO:0042277"
}